{
  "gene_symbol": "CPNE9",
  "term_label": "cellular response to calcium ion",
  "gene_name": "Copine-9",
  "term_id": "GO:0071277",
  "gene": "UniProtKB:Q8IYJ1"
}